{
  "gene_name": "Zinc finger protein 468",
  "term_id": "GO:0000978",
  "gene_symbol": "ZNF468",
  "gene": "UniProtKB:Q5VIY5",
  "term_label": "RNA polymerase II cis-regulatory region sequence-specific DNA binding"
}